regulation of cholesterol metabolic process [GO:0090181] (biological process) Subtypes: regulation of cholesterol biosynthetic process [GO:0045540], positive regulation of cholesterol metabolic process [GO:0090205], negative regulation of cholesterol metabolic process [GO:0090206] Sources: GOC:BHF, GOC:dph, GOC:tb Definition: Any process that modulates the rate, frequency, or extent of cholesterol metabolism, the chemical reactions and pathways involving cholesterol, cholest-5-en-3 beta-ol, the principal sterol of vertebrates and the precursor of many steroids, including bile acids and steroid hormones. Relationships: is a type of GO:0019218; is a type of regulation of small molecule metabolic process [GO:0062012]; regulates GO:0008203